{
  "term_id": "UNKNOWN:0002",
  "gene_name": "Probable G-protein coupled receptor 27",
  "term_label": "Unknown biological process",
  "gene": "UniProtKB:Q9NS67",
  "gene_symbol": "GPR27"
}